{
  "gene_name": "Protocadherin alpha-4",
  "gene": "UniProtKB:Q9UN74",
  "gene_symbol": "PCDHA4",
  "term_id": "GO:0005886",
  "term_label": "plasma membrane"
}